urate oxidase activity [GO:0004846] (molecular function) Definition: Catalysis of the reaction: urate + O2 + H2O = 5-hydroxyisourate + hydrogen peroxide. Sources: EC:1.7.3.3 Also known as: uricase II activity, urate:oxygen oxidoreductase activity, uric acid oxidase activity, uricase activity Relationships: is a type of GO:0016663